growth plate cartilage morphogenesis [GO:0003422] (biological process) Definition: The process in which the anatomical structures of growth plate cartilage are generated and organized. Sources: GOC:ascb_2009, GOC:dph, GOC:tb Relationships: is a type of cartilage morphogenesis [GO:0060536]; is part of GO:0003417 Subtypes: growth plate cartilage chondrocyte morphogenesis [GO:0003429]